{
  "gene_name": "Spermatid nuclear transition protein 1",
  "gene_symbol": "TNP1",
  "term_id": "GO:0007290",
  "term_label": "spermatid nucleus elongation",
  "gene": "UniProtKB:P09430"
}